{
  "gene_symbol": "LINC02693",
  "term_label": "Unknown molecular function",
  "gene": "UniProtKB:A8MQB3",
  "term_id": "UNKNOWN:0001",
  "gene_name": "Putative uncharacterized protein LINC02693"
}